interleukin-17 production [GO:0032620] (biological process) Definition: The appearance of any member of the interleukin-17 family of cytokines due to biosynthesis or secretion following a cellular stimulus, resulting in an increase in its intracellular or extracellular levels. Also known as: CTLA-8 production, Cytotoxic T-lymphocyte-associated antigen 8 production, IL-17 production, interleukin-17 biosynthetic process, interleukin-17 secretion Relationships: is a type of cytokine production [GO:0001816] Sources: GOC:mah, GOC:rv, Wikipedia:Interleukin_17 Regulation: regulated by regulation of interleukin-17 production [GO:0032660]; negatively regulated by negative regulation of interleukin-17 production [GO:0032700]; positively regulated by positive regulation of interleukin-17 production [GO:0032740] Subtypes: interleukin-17A production [GO:0097087], GO:0097088